{
  "term_id": "GO:0005525",
  "gene": "UniProtKB:P61019",
  "gene_symbol": "RAB2A",
  "gene_name": "Ras-related protein Rab-2A",
  "term_label": "GTP binding"
}